{
  "gene_name": "Adenylate kinase 7",
  "term_label": "nucleoside diphosphate kinase activity",
  "gene": "UniProtKB:Q96M32",
  "gene_symbol": "AK7",
  "term_id": "GO:0004550"
}